{
  "gene_symbol": "ZP3",
  "term_label": "acrosin binding",
  "gene_name": "Zona pellucida sperm-binding protein 3",
  "term_id": "GO:0032190",
  "gene": "UniProtKB:P21754"
}